{
  "gene": "UniProtKB:Q5JR59",
  "gene_symbol": "MTUS2",
  "gene_name": "Microtubule-associated tumor suppressor candidate 2",
  "term_label": "Unknown biological process",
  "term_id": "UNKNOWN:0002"
}